lipid droplet transport along microtubule [GO:0031887] (biological process) Relationships: is a type of GO:0072384 Definition: The directed movement of a lipid droplet along a microtubule, mediated by motor proteins. References: PMID:9491895 Also known as: adiposome transport along microtubule, lipid body transport along microtubule, lipid particle transport along microtubule